ribonucleotide metabolic process [GO:0009259] (biological process) Definition: The chemical reactions and pathways involving a ribonucleotide, a compound consisting of ribonucleoside (a base linked to a ribose sugar) esterified with a phosphate group at either the 3' or 5'-hydroxyl group of the sugar. Sources: GOC:go_curators, ISBN:0198506732 Subtypes: purine ribonucleotide metabolic process [GO:0009150], pyrimidine ribonucleotide metabolic process [GO:0009218], ribonucleotide biosynthetic process [GO:0009260], ribonucleotide catabolic process [GO:0009261], FMN metabolic process [GO:0046444] Relationships: is a type of nucleotide metabolic process [GO:0009117]; is a type of GO:0019693 Also known as: ribonucleotide metabolism